{
  "gene": "UniProtKB:Q9UBW5",
  "term_id": "GO:0097320",
  "gene_symbol": "BIN2",
  "term_label": "plasma membrane tubulation",
  "gene_name": "Bridging integrator 2"
}